sensory organ precursor cell fate determination [GO:0016360] (biological process) Definition: The process in which a cell becomes capable of differentiating autonomously into a sensory organ precursor cell regardless of its environment; upon determination, the cell fate cannot be reversed. Relationships: is a type of cell fate determination involved in pattern specification [GO:0060582]; is part of sensory organ boundary specification [GO:0008052] Also known as: sense organ precursor cell fate determination Sources: GOC:go_curators